{
  "gene_name": "Secreted frizzled-related protein 4",
  "term_id": "GO:0005615",
  "gene_symbol": "SFRP4",
  "gene": "UniProtKB:Q6FHJ7",
  "term_label": "extracellular space"
}